{
  "gene_name": "Male-specific lethal 3 homolog",
  "gene": "UniProtKB:Q8N5Y2",
  "gene_symbol": "MSL3",
  "term_label": "Unknown biological process",
  "term_id": "UNKNOWN:0002"
}